{
  "term_label": "spindle assembly",
  "term_id": "GO:0051225",
  "gene": "UniProtKB:Q96CW5",
  "gene_name": "Gamma-tubulin complex component 3",
  "gene_symbol": "TUBGCP3"
}